{
  "gene_name": "Small proline-rich protein 2F",
  "gene": "UniProtKB:Q96RM1",
  "term_label": "Unknown molecular function",
  "gene_symbol": "SPRR2F",
  "term_id": "UNKNOWN:0001"
}